limb spinous cell fate specification [GO:0060894] (biological process) Definition: The process in which a cell becomes capable of differentiating autonomously into a limb spinous cell in an environment that is neutral with respect to the developmental pathway; upon specification, the cell fate can be reversed. Relationships: is a type of GO:0009957; is a type of cell fate specification involved in pattern specification [GO:0060573]; BFO_0000050 limb epidermis stratification [GO:0060888]; is part of limb spinous cell differentiation [GO:0060890] Sources: GOC:dph, GOC:sdb_2009, GOC:tb